coproporphyrinogen oxidase activity [GO:0004109] (molecular function) Relationships: is a type of GO:0016634 Also known as: coprogen oxidase activity, coproporphyrinogen-III oxidase activity, coproporphyrinogenase activity, coproporphyrinogen:oxygen oxidoreductase (decarboxylating) Sources: EC:1.3.3.3, RHEA:18257 Definition: Catalysis of the reaction: coproporphyrinogen III + 2 H+ + O2 = 2 CO2 + 2 H2O + protoporphyrinogen IX.